lymph gland development [GO:0048542] (biological process) Relationships: is a type of hematopoietic or lymphoid organ development [GO:0048534]; is a type of gland development [GO:0048732] Also known as: haematopoietic organ development, haemopoietic organ development, hematopoietic organ development, hemopoietic organ development Definition: The process whose specific outcome is the progression of the lymph gland over time, from its formation to the mature structure. The lymph gland is one of the sites of hemocyte differentiation. It consists of three to six bilaterally paired lobes that are attached to the cardioblasts during larval stages, and it degenerates during pupal stages. Sources: GOC:mtg_sensu, GOC:rc